aromatic-hydroxylamine O-acetyltransferase activity [GO:0047188] (molecular function) Definition: Catalysis of the reaction: N-hydroxy-4-aminobiphenyl + N-hydroxy-4-acetylaminonbiphenyl = N-acetoxy-4-aminobiphenyl + N-hydroxy-4-aminobiphenyl. Relationships: is a type of GO:0016413 Also known as: N,O-acetyltransferase activity, N-hydroxy-2-acetylaminofluorene N-O acyltransferase activity, N-hydroxy-4-acetylaminobiphenyl:N-hydroxy-4-aminobiphenyl O-acetyltransferase activity, aromatic hydroxylamine acetyltransferase activity, arylhydroxamate acyltransferase activity, arylhydroxamic acid N,O-acetyltransferase activity, arylhydroxamic acyltransferase activity Sources: EC:2.3.1.56, MetaCyc:2.3.1.56-RXN